superoxide dismutase copper chaperone activity [GO:0016532] (molecular function) Relationships: is a type of copper chaperone activity [GO:0016531] Note: See also the molecular function term 'superoxide dismutase activity ; GO:0004784'. References: PMID:15064408, PMID:9295278 Sources: GOC:vw, http://link.springer-ny.com/link/service/journals/00335/papers/0011005/00110409.html Also known as: superoxide dismutase copper carrier activity Definition: A copper chaperone activity that specifically delivers copper to the Cu-Zn superoxide dismutase, to activate superoxide dismutase activity.